TAP binding [GO:0046977] (molecular function) Subtypes: TAP1 binding [GO:0046978], TAP2 binding [GO:0046979] Relationships: is a type of protein binding [GO:0005515] References: PMID:11133832 Definition: Binding to TAP protein, transporter associated with antigen processing protein. TAP protein is a heterodimeric peptide transporter consisting of the subunits TAP1 and TAP2.